{
  "gene_symbol": "INTS13",
  "gene": "UniProtKB:Q9NVM9",
  "gene_name": "Integrator complex subunit 13",
  "term_label": "centrosome localization",
  "term_id": "GO:0051642"
}